{
  "term_id": "GO:0008201",
  "gene_name": "Leucine-rich repeat-containing G-protein coupled receptor 6",
  "gene": "UniProtKB:Q9HBX8",
  "term_label": "heparin binding",
  "gene_symbol": "LGR6"
}